{
  "gene_symbol": "ZNF217",
  "gene": "UniProtKB:O75362",
  "term_id": "GO:0000981",
  "term_label": "DNA-binding transcription factor activity, RNA polymerase II-specific",
  "gene_name": "Zinc finger protein 217"
}